B cell chemotaxis [GO:0035754] (biological process) Regulation: regulated by GO:2000537; positively regulated by positive regulation of B cell chemotaxis [GO:2000538]; RO_0002212 by negative regulation of B cell chemotaxis [GO:2000550] Relationships: is a type of lymphocyte chemotaxis [GO:0048247] Subtypes: B cell chemotaxis across high endothelial venule [GO:0035769] Sources: CL:0000236, GOC:BHF Definition: The directed movement of a B cell guided by a specific chemical concentration gradient. Movement may be towards a higher concentration (positive chemotaxis) or towards a lower concentration (negative chemotaxis).